{
  "term_id": "GO:0005794",
  "term_label": "Golgi apparatus",
  "gene": "UniProtKB:O14735",
  "gene_name": "CDP-diacylglycerol--inositol 3-phosphatidyltransferase",
  "gene_symbol": "CDIPT"
}